{
  "term_label": "signaling receptor binding",
  "gene": "UniProtKB:Q6UXG8",
  "term_id": "GO:0005102",
  "gene_name": "Butyrophilin-like protein 9",
  "gene_symbol": "BTNL9"
}